regulation of hyaluronan biosynthetic process [GO:1900125] (biological process) Subtypes: negative regulation of hyaluronan biosynthetic process [GO:1900126], positive regulation of hyaluronan biosynthetic process [GO:1900127] Relationships: is a type of regulation of polysaccharide biosynthetic process [GO:0032885]; regulates hyaluronan biosynthetic process [GO:0030213] Also known as: regulation of hyaluronan anabolism, regulation of hyaluronan biosynthesis, regulation of hyaluronan formation, regulation of hyaluronan synthesis Definition: Any process that modulates the frequency, rate or extent of hyaluronan biosynthetic process. Sources: GOC:TermGenie, GOC:yaf